regulation of microtubule polymerization or depolymerization [GO:0031110] (biological process) Definition: Any process that modulates the frequency, rate or extent of microtubule polymerization or depolymerization by the addition or removal of tubulin heterodimers from a microtubule. Sources: GOC:mah Subtypes: negative regulation of microtubule polymerization or depolymerization [GO:0031111], GO:0031112, regulation of microtubule polymerization [GO:0031113], regulation of microtubule depolymerization [GO:0031114] Relationships: is a type of regulation of microtubule cytoskeleton organization [GO:0070507]; regulates microtubule polymerization or depolymerization [GO:0031109]